{
  "gene_symbol": "NFKBIZ",
  "gene_name": "NF-kappa-B inhibitor zeta",
  "term_label": "nucleus",
  "gene": "UniProtKB:Q9BYH8",
  "term_id": "GO:0005634"
}